{
  "gene": "UniProtKB:Q4VC39",
  "term_label": "Unknown molecular function",
  "term_id": "UNKNOWN:0001",
  "gene_name": "Putative HIG1 domain family member 2B",
  "gene_symbol": "HIGD2B"
}